{
  "gene_symbol": "TRAJ29",
  "term_id": "UNKNOWN:0001",
  "gene_name": "T cell receptor alpha joining 29 (Fragment)",
  "term_label": "Unknown molecular function",
  "gene": "UniProtKB:A0A075B711"
}